{
  "gene_name": "Melanopsin",
  "term_id": "GO:0007186",
  "gene": "UniProtKB:Q9UHM6",
  "term_label": "G protein-coupled receptor signaling pathway",
  "gene_symbol": "OPN4"
}